lymphocyte apoptotic process [GO:0070227] (biological process) Relationships: is a type of leukocyte apoptotic process [GO:0071887] Note: Note that a lymphocyte is a cell of the B cell, T cell, or natural killer cell lineage (CL:0000542). Sources: CL:0000542, GOC:add, GOC:mtg_apoptosis, ISBN:0781765196 Regulation: regulated by regulation of lymphocyte apoptotic process [GO:0070228]; negatively regulated by negative regulation of lymphocyte apoptotic process [GO:0070229]; positively regulated by positive regulation of lymphocyte apoptotic process [GO:0070230] Definition: Any apoptotic process in a lymphocyte, a leukocyte commonly found in the blood and lymph that has the characteristics of a large nucleus, a neutral staining cytoplasm, and prominent heterochromatin. Also known as: lymphocyte apoptosis Subtypes: B cell apoptotic process [GO:0001783], T cell apoptotic process [GO:0070231], natural killer cell apoptotic process [GO:0070246]